{
  "gene_symbol": "SPESP1",
  "term_label": "Unknown molecular function",
  "term_id": "UNKNOWN:0001",
  "gene_name": "Sperm equatorial segment protein 1",
  "gene": "UniProtKB:Q6UW49"
}